{
  "term_label": "mediator complex",
  "term_id": "GO:0016592",
  "gene_symbol": "MED19",
  "gene": "UniProtKB:A0JLT2",
  "gene_name": "Mediator of RNA polymerase II transcription subunit 19"
}